{
  "gene": "UniProtKB:P52948",
  "gene_name": "Nuclear pore complex protein Nup98-Nup96",
  "gene_symbol": "NUP98",
  "term_id": "GO:0000973",
  "term_label": "post-transcriptional tethering of RNA polymerase II gene DNA at nuclear periphery"
}